{
  "gene": "UniProtKB:P35222",
  "term_id": "GO:0045296",
  "gene_symbol": "CTNNB1",
  "gene_name": "Catenin beta-1",
  "term_label": "cadherin binding"
}